{
  "term_id": "GO:0006260",
  "term_label": "DNA replication",
  "gene": "UniProtKB:P11387",
  "gene_symbol": "TOP1",
  "gene_name": "DNA topoisomerase 1"
}